mating type region replication fork barrier binding [GO:1990943] (molecular function) References: PMID:18723894 Relationships: is a type of replication fork barrier binding [GO:0031634] Definition: Binding to the replication fork barrier found in the mating type region of fission yeast. Also known as: RTS1 barrier binding, RTS1 element binding